{
  "term_id": "GO:0000981",
  "gene_symbol": "MGA",
  "gene_name": "MAX gene-associated protein",
  "gene": "UniProtKB:Q8IWI9",
  "term_label": "DNA-binding transcription factor activity, RNA polymerase II-specific"
}